{
  "term_label": "Unknown cellular component",
  "gene_name": "Proteasome assembly chaperone 4",
  "gene": "UniProtKB:Q5JS54",
  "gene_symbol": "PSMG4",
  "term_id": "UNKNOWN:0003"
}